{
  "gene": "UniProtKB:Q01629",
  "gene_symbol": "IFITM2",
  "gene_name": "Interferon-induced transmembrane protein 2",
  "term_id": "GO:0035455",
  "term_label": "response to interferon-alpha"
}